negative regulation of early stripe melanocyte differentiation [GO:0050947] (biological process) Relationships: is a type of GO:0045635; is_a regulation of early stripe melanocyte differentiation [GO:0050939]; negatively regulates early stripe melanocyte differentiation [GO:0050933] Also known as: down regulation of early stripe melanocyte differentiation, down-regulation of early stripe melanocyte differentiation, downregulation of early stripe melanocyte differentiation, negative regulation of early stripe melanophore differentiation, inhibition of early stripe melanocyte differentiation Definition: Any process that stops, prevents, or reduces the frequency, rate or extent of early stripe melanocyte differentiation. Sources: GOC:ai